N-benzoyl-L-glutamate synthetase activity [GO:0052626] (molecular function) Also known as: benzoate amino acid synthetase activity, benzoyl amino acid synthetase activity Relationships: is a type of acid-amino acid ligase activity [GO:0016881] References: PMID:19189963 Sources: MetaCyc:RXN-10886 Definition: Catalysis of the reaction: benzoate + L-glutamate + ATP = N-benzoyl-L-glutamate + AMP + diphosphate + H+.